{
  "term_label": "telomere maintenance",
  "gene": "UniProtKB:O60921",
  "term_id": "GO:0000723",
  "gene_name": "Checkpoint protein HUS1",
  "gene_symbol": "HUS1"
}